{
  "gene_name": "Endothelial cell-selective adhesion molecule",
  "gene_symbol": "ESAM",
  "gene": "UniProtKB:Q96AP7",
  "term_id": "GO:0007156",
  "term_label": "homophilic cell-cell adhesion"
}